mRNA localization resulting in post-transcriptional regulation of gene expression [GO:0010609] (biological process) Sources: GOC:dph, GOC:tb Relationships: is a type of intracellular mRNA localization [GO:0008298]; is a type of post-transcriptional regulation of gene expression [GO:0010608] Also known as: mRNA localisation resulting in posttranscriptional regulation of gene expression, mRNA localization resulting in posttranscriptional regulation of gene expression, posttranscriptional regulation of gene expression by mRNA localisation, posttranscriptional regulation of gene expression by mRNA localization Definition: Any process that modulates the frequency, rate or extent of gene expression after the production of a mRNA transcript by its transport into, or maintenance in, a specific location within the cell.